{
  "term_id": "GO:0002322",
  "gene_name": "CD180 antigen",
  "gene": "UniProtKB:Q99467",
  "term_label": "B cell proliferation involved in immune response",
  "gene_symbol": "CD180"
}